{
  "term_label": "cell-cell junction",
  "gene_symbol": "FRMD6",
  "term_id": "GO:0005911",
  "gene": "UniProtKB:Q96NE9",
  "gene_name": "FERM domain-containing protein 6"
}